dorsal spinal cord interneuron axon guidance [GO:0097378] (biological process) Definition: The process in which the migration of an axon growth cone of a dorsal spinal cord interneuron is directed to a specific target site in response to a combination of attractive and repulsive cues. A dorsal spinal cord interneuron is an interneuron located in the dorsal part of the spinal cord. Sources: GOC:yaf Also known as: dorsal interneuron axon guidance Relationships: is a type of GO:0097377 Subtypes: dorsal spinal cord interneuron posterior axon guidance [GO:0097379], dorsal spinal cord interneuron anterior axon guidance [GO:0097380]